ribonuclease inhibitor activity [GO:0008428] (molecular function) Sources: GOC:ai Relationships: is a type of nuclease inhibitor activity [GO:0140721]; negatively regulates RNA nuclease activity [GO:0004540] Definition: Binds to and stops, prevents or reduces the activity of ribonuclease. Subtypes: endoribonuclease inhibitor activity [GO:0060698] Also known as: RNA nuclease inhibitor activity